{
  "term_label": "cytoplasm",
  "gene_symbol": "USP49",
  "gene_name": "Ubiquitin carboxyl-terminal hydrolase 49",
  "gene": "UniProtKB:Q70CQ1",
  "term_id": "GO:0005737"
}